{
  "term_label": "serine-type endopeptidase activity",
  "gene": "UniProtKB:P00734",
  "term_id": "GO:0004252",
  "gene_symbol": "F2",
  "gene_name": "Prothrombin"
}